{
  "term_label": "histone H3K4me/H3K4me2/H3K4me3 demethylase activity",
  "gene": "UniProtKB:P41229",
  "gene_name": "Lysine-specific demethylase 5C",
  "gene_symbol": "KDM5C",
  "term_id": "GO:0034647"
}